{
  "term_id": "GO:0017040",
  "term_label": "N-acylsphingosine amidohydrolase activity",
  "gene_name": "Acid ceramidase",
  "gene": "UniProtKB:Q13510",
  "gene_symbol": "ASAH1"
}